{
  "term_id": "UNKNOWN:0001",
  "gene_name": "Filaggrin-2",
  "gene_symbol": "FLG2",
  "term_label": "Unknown molecular function",
  "gene": "UniProtKB:Q5D862"
}